{
  "gene_symbol": "NOS2",
  "term_id": "GO:0032496",
  "gene_name": "Nitric oxide synthase, inducible",
  "gene": "UniProtKB:P35228",
  "term_label": "response to lipopolysaccharide"
}